{
  "gene_name": "Carboxypeptidase A1",
  "gene": "UniProtKB:P15085",
  "gene_symbol": "CPA1",
  "term_label": "metallocarboxypeptidase activity",
  "term_id": "GO:0004181"
}